negative regulation of juvenile hormone biosynthetic process [GO:0045968] (biological process) Also known as: down regulation of juvenile hormone biosynthetic process, down-regulation of juvenile hormone biosynthetic process, downregulation of juvenile hormone biosynthetic process, negative regulation of juvenile hormone anabolism, negative regulation of juvenile hormone biosynthesis, negative regulation of juvenile hormone formation, negative regulation of juvenile hormone synthesis, inhibition of juvenile hormone biosynthetic process Sources: GOC:go_curators Definition: Any process that stops, prevents, or reduces the frequency, rate or extent of the chemical reactions and pathways resulting in the formation of juvenile hormone. Relationships: is_a regulation of juvenile hormone biosynthetic process [GO:0007557]; is a type of negative regulation of hormone biosynthetic process [GO:0032353]; is a type of GO:0045928; is a type of negative regulation of lipid biosynthetic process [GO:0051055]; negatively regulates GO:0006718